{
  "gene_name": "Endothelial transcription factor GATA-2",
  "gene": "UniProtKB:P23769",
  "term_id": "GO:0000981",
  "term_label": "DNA-binding transcription factor activity, RNA polymerase II-specific",
  "gene_symbol": "GATA2"
}